{
  "term_id": "GO:0016064",
  "gene_name": "Immunoglobulin heavy variable 1_OR15-9 (non-functional) (Fragment)",
  "term_label": "immunoglobulin mediated immune response",
  "gene_symbol": "IGHV1OR15-9",
  "gene": "UniProtKB:A0A0B4J2B8"
}